{
  "gene": "UniProtKB:O75324",
  "gene_name": "Stannin",
  "gene_symbol": "SNN",
  "term_id": "UNKNOWN:0002",
  "term_label": "Unknown biological process"
}